type 1 parathyroid hormone receptor binding [GO:0031857] (molecular function) Sources: GOC:mah, GOC:nln Also known as: type 1 parathyroid hormone receptor ligand Definition: Binding to a type 1 parathyroid hormone receptor. Relationships: is a type of GO:0031856